{
  "gene_name": "Zinc finger protein 354C",
  "term_label": "nucleus",
  "gene_symbol": "ZNF354C",
  "gene": "UniProtKB:Q86Y25",
  "term_id": "GO:0005634"
}